{
  "gene": "UniProtKB:P19174",
  "term_label": "ruffle membrane",
  "term_id": "GO:0032587",
  "gene_name": "1-phosphatidylinositol 4,5-bisphosphate phosphodiesterase gamma-1",
  "gene_symbol": "PLCG1"
}